{
  "gene_name": "Glutamine--fructose-6-phosphate aminotransferase [isomerizing] 1",
  "gene_symbol": "GFPT1",
  "term_label": "UDP-N-acetylglucosamine metabolic process",
  "term_id": "GO:0006047",
  "gene": "UniProtKB:Q06210"
}